{
  "gene_symbol": "MARCHF4",
  "term_label": "trans-Golgi network",
  "gene": "UniProtKB:Q9P2E8",
  "term_id": "GO:0005802",
  "gene_name": "E3 ubiquitin-protein ligase MARCHF4"
}